channel-forming ionophore activity [GO:0022886] (molecular function) Definition: Enables transport of a solute across a membrane. This kind of transporter interacts much more weakly with the solute than the carrier does. It is an aqueous pore that extends across the membrane. It may change from closed to open and back. It transports faster than a carrier. It is always passive. Sources: GOC:mtg_transport, ISBN:0815340729 Also known as: ionophore activity Relationships: is_a channel activity [GO:0015267]